{
  "term_id": "GO:0004252",
  "gene_name": "Acylamino-acid-releasing enzyme",
  "term_label": "serine-type endopeptidase activity",
  "gene": "UniProtKB:P13798",
  "gene_symbol": "APEH"
}